{
  "gene": "UniProtKB:P12956",
  "term_id": "GO:0006303",
  "gene_name": "X-ray repair cross-complementing protein 6",
  "term_label": "double-strand break repair via nonhomologous end joining",
  "gene_symbol": "XRCC6"
}